{
  "gene_name": "Tubulin monoglycylase TTLL3",
  "term_label": "protein-glycine ligase activity, initiating",
  "gene_symbol": "TTLL3",
  "term_id": "GO:0070736",
  "gene": "UniProtKB:Q9Y4R7"
}